{
  "gene_name": "Glycosaminoglycan xylosylkinase",
  "gene_symbol": "FAM20B",
  "term_id": "UNKNOWN:0003",
  "term_label": "Unknown cellular component",
  "gene": "UniProtKB:O75063"
}